{
  "gene": "UniProtKB:P08238",
  "gene_symbol": "HSP90AB1",
  "term_id": "GO:0050821",
  "gene_name": "Heat shock protein HSP 90-beta",
  "term_label": "protein stabilization"
}